{
  "term_id": "GO:0006816",
  "gene_name": "Transient receptor potential cation channel subfamily M member 1",
  "gene": "UniProtKB:Q7Z4N2",
  "term_label": "calcium ion transport",
  "gene_symbol": "TRPM1"
}